{
  "term_id": "GO:0005912",
  "gene": "UniProtKB:Q9HBT6",
  "gene_symbol": "CDH20",
  "term_label": "adherens junction",
  "gene_name": "Cadherin-20"
}